single-stranded 3'-5' DNA helicase activity [GO:1990518] (molecular function) Relationships: is a type of single-stranded DNA helicase activity [GO:0017116]; is a type of 3'-5' DNA helicase activity [GO:0043138] References: PMID:25165823 Definition: Catalysis of the reaction: ATP + H2O = ADP + phosphate, in the presence of single-stranded DNA; drives the unwinding of the DNA helix in the direction 3' to 5'.